phenylalanine-tRNA ligase complex [GO:0009328] (cellular component) References: PMID:20223217 Definition: An enzyme complex that catalyzes the ligation of phenylalanine to tRNA(Phe), forming L-phenylalanyl-tRNA(Phe). Relationships: is a type of GO:1902494; is part of cytoplasm [GO:0005737]